{
  "gene": "UniProtKB:Q9UMS4",
  "gene_name": "Pre-mRNA-processing factor 19",
  "term_label": "Prp19 complex",
  "term_id": "GO:0000974",
  "gene_symbol": "PRPF19"
}